regulation of asperfuranone biosynthetic process [GO:1900637] (BP) Sources: GOC:TermGenie, GOC:di Definition: Any process that modulates the frequency, rate or extent of asperfuranone biosynthetic process. Relationships: is a type of GO:1900732; is a type of regulation of alcohol biosynthetic process [GO:1902930]; regulates asperfuranone biosynthetic process [GO:1900554] Subtypes: negative regulation of asperfuranone biosynthetic process [GO:1900638], positive regulation of asperfuranone biosynthetic process [GO:1900639] Also known as: regulation of asperfuranone anabolism, regulation of asperfuranone biosynthesis, regulation of asperfuranone formation, regulation of asperfuranone synthesis